establishment of Golgi localization [GO:0051683] (biological process) Sources: GOC:ai Also known as: establishment of Golgi apparatus localization, establishment of Golgi body localization, establishment of Golgi localisation Relationships: is a type of Golgi localization [GO:0051645]; is a type of establishment of localization in cell [GO:0051649]; is a type of establishment of organelle localization [GO:0051656] Definition: The directed movement of the Golgi to a specific location.